positive regulation of response to calcium ion [GO:1905947] (biological process) Definition: Any process that activates or increases the frequency, rate or extent of response to calcium ion. Relationships: is a type of positive regulation of response to stimulus [GO:0048584]; is_a regulation of response to calcium ion [GO:1905945]; positively regulates response to calcium ion [GO:0051592] References: PMID:11404397 Sources: GOC:TermGenie, GOC:aruk, GOC:bc, GO_REF:0000058 Also known as: positive regulation of response to Ca2+ ion, up regulation of response to Ca2+ ion, up regulation of response to calcium ion, up-regulation of response to Ca2+ ion, up-regulation of response to calcium ion, upregulation of response to Ca2+ ion, upregulation of response to calcium ion, activation of response to Ca2+ ion, activation of response to calcium ion